{
  "term_id": "GO:0051045",
  "gene_symbol": "TIMP2",
  "gene": "UniProtKB:P16035",
  "gene_name": "Metalloproteinase inhibitor 2",
  "term_label": "negative regulation of membrane protein ectodomain proteolysis"
}